{
  "term_label": "RNA helicase activity",
  "gene_name": "Probable ATP-dependent RNA helicase DDX5",
  "gene_symbol": "DDX5",
  "term_id": "GO:0003724",
  "gene": "UniProtKB:P17844"
}